{
  "gene_symbol": "OR8B8",
  "term_id": "GO:0005549",
  "gene_name": "Olfactory receptor 8B8",
  "term_label": "odorant binding",
  "gene": "UniProtKB:Q15620"
}